negative regulation of corticotropin-releasing hormone receptor activity [GO:1900011] (biological process) References: PMID:18234674 Sources: GOC:TermGenie, GOC:yaf Also known as: down regulation of CRF receptor activity, down regulation of CRH receptor activity, down regulation of adrenocorticotropin-releasing hormone receptor activity, down regulation of corticotropin-releasing factor receptor activity, negative regulation of CRF receptor activity, negative regulation of CRH receptor activity, negative regulation of adrenocorticotropin-releasing hormone receptor activity, negative regulation of corticotropin-releasing factor receptor activity, down regulation of corticotropin-releasing hormone receptor activity Definition: Any process that stops, prevents or reduces the frequency, rate or extent of corticotropin-releasing hormone receptor activity. Relationships: is a type of negative regulation of signal transduction [GO:0009968]; is_a GO:2000272; RO_0002212 corticotropin-releasing hormone receptor activity [GO:0043404]